{
  "term_id": "GO:0015937",
  "gene": "UniProtKB:Q9HAB8",
  "term_label": "coenzyme A biosynthetic process",
  "gene_symbol": "PPCS",
  "gene_name": "Phosphopantothenate--cysteine ligase"
}